{
  "term_id": "UNKNOWN:0001",
  "gene": "UniProtKB:P34810",
  "term_label": "Unknown molecular function",
  "gene_symbol": "CD68",
  "gene_name": "Macrosialin"
}